{
  "gene_name": "WD and tetratricopeptide repeats protein 1",
  "gene_symbol": "WDTC1",
  "term_id": "GO:0005737",
  "gene": "UniProtKB:Q8N5D0",
  "term_label": "cytoplasm"
}